protein refolding [GO:0042026] (biological process) Regulation: RO_0002211 by regulation of protein refolding [GO:0061083]; negatively regulated by negative regulation of protein refolding [GO:0061084]; positively regulated by positive regulation of protein refolding [GO:1904592] Relationships: is a type of protein folding [GO:0006457] Sources: GOC:mb Also known as: heat shock protein activity Definition: The process carried out by a cell that restores the biological activity of an unfolded or misfolded protein, using helper proteins such as chaperones.